{
  "gene_name": "Polycomb protein EED",
  "gene_symbol": "EED",
  "term_label": "negative regulation of transcription by RNA polymerase II",
  "gene": "UniProtKB:O75530",
  "term_id": "GO:0000122"
}